{
  "gene_symbol": "SLC8A1",
  "gene": "UniProtKB:P32418",
  "gene_name": "Sodium_calcium exchanger 1",
  "term_label": "axon",
  "term_id": "GO:0030424"
}